DNA polymerase activity [GO:0034061] (MF) Subtypes: DNA-directed DNA polymerase activity [GO:0003887], DNA nucleotidylexotransferase activity [GO:0003912], GO:0003964 Sources: RHEA:22508 Regulation: positively regulated by DNA polymerase processivity factor activity [GO:0030337] Relationships: is a type of GO:0016779; is a type of catalytic activity, acting on DNA [GO:0140097]; is part of DNA biosynthetic process [GO:0071897] Definition: Catalysis of the reaction: a 2'-deoxyribonucleoside 5'-triphosphate + DNA(n) = diphosphate + DNA(n+1).